{
  "gene_symbol": "UCHL3",
  "term_label": "cysteine-type deubiquitinase activity",
  "term_id": "GO:0004843",
  "gene": "UniProtKB:P15374",
  "gene_name": "Ubiquitin carboxyl-terminal hydrolase isozyme L3"
}